{
  "term_id": "GO:0034056",
  "gene_symbol": "ESR2",
  "gene": "UniProtKB:Q92731",
  "term_label": "estrogen response element binding",
  "gene_name": "Estrogen receptor beta"
}